{
  "term_id": "GO:0003847",
  "gene_name": "Platelet-activating factor acetylhydrolase",
  "gene": "UniProtKB:Q13093",
  "term_label": "1-alkyl-2-acetylglycerophosphocholine esterase activity",
  "gene_symbol": "PLA2G7"
}